multicellular organism development [GO:0007275] (biological process) Definition: The biological process whose specific outcome is the progression of a multicellular organism over time from an initial condition (e.g. a zygote or a young adult) to a later condition (e.g. a multicellular animal or an aged adult). Note: Note that this term was 'developmental process'. Regulation: RO_0002211 by GO:2000026 Subtypes: larval development [GO:0002164], instar larval or pupal development [GO:0002165], metamorphosis [GO:0007552], embryo development [GO:0009790], gametophyte development [GO:0048229] Relationships: is a type of multicellular organismal process [GO:0032501]; is a type of anatomical structure development [GO:0048856] Sources: GOC:dph, GOC:ems, GOC:isa_complete, GOC:tb